{
  "gene": "UniProtKB:O95639",
  "gene_name": "Cleavage and polyadenylation specificity factor subunit 4",
  "term_label": "Unknown biological process",
  "gene_symbol": "CPSF4",
  "term_id": "UNKNOWN:0002"
}